{
  "gene_symbol": "ELOVL6",
  "gene": "UniProtKB:Q9H5J4",
  "gene_name": "Elongation of very long chain fatty acids protein 6",
  "term_label": "fatty acid elongation, polyunsaturated fatty acid",
  "term_id": "GO:0034626"
}